aldosterone secretion [GO:0035932] (biological process) Regulation: regulated by regulation of aldosterone secretion [GO:2000858]; negatively regulated by GO:2000859; positively regulated by positive regulation of aldosterone secretion [GO:2000860] Definition: The regulated release of aldosterone into the circulatory system. Aldosterone is a pregnane-based steroid hormone produced by the outer-section (zona glomerulosa) of the adrenal cortex in the adrenal gland, and acts on the distal tubules and collecting ducts of the kidney to cause the conservation of sodium, secretion of potassium, increased water retention, and increased blood pressure. The overall effect of aldosterone is to increase reabsorption of ions and water in the kidney. Sources: GOC:sl Relationships: is_a organic hydroxy compound transport [GO:0015850]; is a type of mineralocorticoid secretion [GO:0035931]